 [go#goslim:pombe] Note: Fission yeast GO slim